{
  "term_id": "UNKNOWN:0001",
  "term_label": "Unknown molecular function",
  "gene_symbol": "FAM47E",
  "gene_name": "Protein FAM47E",
  "gene": "UniProtKB:Q6ZV65"
}